sarcoglycan complex [GO:0016012] (cellular component) Definition: A protein complex formed of four sarcoglycans plus sarcospan; there are six known sarcoglycans: alpha-, beta-, gamma-, delta-, epsilon- and zeta-sarcoglycan; all are N-glycosylated single-pass transmembrane proteins. The sarcoglycan-sarcospan complex is a subcomplex of the dystrophin glycoprotein complex, and is fixed to the dystrophin axis by a lateral association with the dystroglycan complex. Relationships: is a type of plasma membrane protein complex [GO:0098797]; is part of dystroglycan complex [GO:0016011] References: PMID:15117830, PMID:16710609 Also known as: sarcoglycan-sarcospan complex